{
  "term_id": "GO:0006357",
  "gene_symbol": "TCF4",
  "gene": "UniProtKB:P15884",
  "gene_name": "Transcription factor 4",
  "term_label": "regulation of transcription by RNA polymerase II"
}